{
  "gene_symbol": "TRIM49C",
  "gene": "UniProtKB:P0CI26",
  "term_label": "regulation of gene expression",
  "term_id": "GO:0010468",
  "gene_name": "Tripartite motif-containing protein 49C"
}